endosperm protein body [GO:0042735] (cellular component) References: PMID:7704047 Sources: GOC:jl Definition: A membrane-bounded plant organelle found in the developing endosperm, contains storage proteins. Relationships: is a type of GO:0043231; is part of GO:0005737